{
  "gene": "UniProtKB:Q01113",
  "gene_name": "Interleukin-9 receptor",
  "gene_symbol": "IL9R",
  "term_id": "GO:0009897",
  "term_label": "external side of plasma membrane"
}